{
  "gene_name": "Transmembrane protein 208",
  "gene_symbol": "TMEM208",
  "term_id": "GO:0006624",
  "term_label": "vacuolar protein processing",
  "gene": "UniProtKB:Q9BTX3"
}